{
  "gene_name": "Thymosin beta-10",
  "term_label": "actin monomer binding",
  "term_id": "GO:0003785",
  "gene": "UniProtKB:P63313",
  "gene_symbol": "TMSB10"
}